eating behavior [GO:0042755] (biological process) Relationships: is a type of feeding behavior [GO:0007631] Regulation: regulated by regulation of eating behavior [GO:1903998]; negatively regulated by negative regulation of eating behavior [GO:1903999]; positively regulated by positive regulation of eating behavior [GO:1904000] Subtypes: reduction of food intake in response to dietary excess [GO:0002023], nematode pharyngeal pumping [GO:0043050] Also known as: eating behaviour Definition: The specific behavior of an organism relating to the intake of food, any substance (usually solid) that can be metabolized by an organism to give energy and build tissue. References: PMID:19361967 Sources: GOC:jl, GOC:pr